adenine import across plasma membrane [GO:0098702] (biological process) Also known as: adenine import into cell Relationships: is a type of adenine transport [GO:0015853]; is a type of import across plasma membrane [GO:0098739]; is a type of purine nucleobase transmembrane transport [GO:1904823] Sources: GOC:dos Definition: The directed movement of adenine from outside of a cell, across the plasma membrane and into the cytosol.